endoplasmic reticulum cisternal network maintenance [GO:0071785] (biological process) Definition: The organization process that preserves the endoplasmic reticulum (ER) cisternal network in a stable functional or structural state. The ER cisternal network is the ER part that comprises the membranes with low curvature in cross-section. Also known as: ER cisternal network maintenance Relationships: is a type of cellular component maintenance [GO:0043954]; is a type of GO:0071783 References: PMID:16469703, PMID:20434336 Sources: GOC:mah